{
  "gene": "UniProtKB:P29597",
  "term_id": "GO:0035556",
  "gene_symbol": "TYK2",
  "gene_name": "Non-receptor tyrosine-protein kinase TYK2",
  "term_label": "intracellular signal transduction"
}